{
  "term_id": "GO:0008574",
  "gene": "UniProtKB:Q96AC6",
  "gene_name": "Kinesin-like protein KIFC2",
  "gene_symbol": "KIFC2",
  "term_label": "plus-end-directed microtubule motor activity"
}